{
  "gene_symbol": "POLR2M",
  "term_label": "I band",
  "gene_name": "DNA-directed RNA polymerase II subunit GRINL1A",
  "term_id": "GO:0031674",
  "gene": "UniProtKB:P0CAP2"
}